{
  "term_id": "GO:0007507",
  "gene": "UniProtKB:Q9NYJ8",
  "gene_symbol": "TAB2",
  "gene_name": "TGF-beta-activated kinase 1 and MAP3K7-binding protein 2",
  "term_label": "heart development"
}